{
  "gene": "UniProtKB:Q9UBH6",
  "gene_symbol": "XPR1",
  "term_label": "plasma membrane",
  "gene_name": "Solute carrier family 53 member 1",
  "term_id": "GO:0005886"
}